{
  "gene": "UniProtKB:Q8WUX2",
  "gene_name": "Glutathione-specific gamma-glutamylcyclotransferase 2",
  "gene_symbol": "CHAC2",
  "term_label": "glutathione catabolic process",
  "term_id": "GO:0006751"
}